{
  "gene": "UniProtKB:Q2M3C6",
  "gene_symbol": "TMEM266",
  "term_label": "plasma membrane",
  "term_id": "GO:0005886",
  "gene_name": "Transmembrane protein 266"
}